{
  "term_label": "regulation of calcium ion-dependent exocytosis",
  "gene_symbol": "SYT8",
  "gene_name": "Synaptotagmin-8",
  "gene": "UniProtKB:Q8NBV8",
  "term_id": "GO:0017158"
}